positive regulation of skeletal muscle tissue development [GO:0048643] (biological process) Also known as: up regulation of skeletal muscle development, up-regulation of skeletal muscle development, upregulation of skeletal muscle development, activation of skeletal muscle development, stimulation of skeletal muscle development Definition: Any process that activates, maintains or increases the rate of skeletal muscle tissue development. Sources: GOC:go_curators Relationships: is a type of GO:0045844; is a type of regulation of skeletal muscle tissue development [GO:0048641]; RO_0002213 GO:0007519 Subtypes: positive regulation of branchiomeric skeletal muscle development [GO:0014712], positive regulation of extraocular skeletal muscle development [GO:0014727], GO:0048633, positive regulation of skeletal muscle fiber development [GO:0048743]